CARD8 inflammasome complex [GO:0140634] (cellular component) Definition: An inflammasome complex that consists of CARD8 and CASP1. Relationships: is a type of canonical inflammasome complex [GO:0061702] References: PMID:33420028, PMID:33420033, PMID:33542150